{
  "gene": "UniProtKB:Q01718",
  "gene_name": "Adrenocorticotropic hormone receptor",
  "term_id": "GO:0004930",
  "gene_symbol": "MC2R",
  "term_label": "G protein-coupled receptor activity"
}